{
  "term_id": "UNKNOWN:0001",
  "gene": "UniProtKB:Q9P1U1",
  "gene_name": "Actin-related protein 3B",
  "term_label": "Unknown molecular function",
  "gene_symbol": "ACTR3B"
}